{
  "gene_symbol": "SRPK3",
  "term_id": "GO:0000245",
  "gene": "UniProtKB:Q9UPE1",
  "gene_name": "SRSF protein kinase 3",
  "term_label": "spliceosomal complex assembly"
}